{
  "gene_name": "Phospholipase A2, membrane associated",
  "gene_symbol": "PLA2G2A",
  "gene": "UniProtKB:P14555",
  "term_label": "phosphatidylglycerol metabolic process",
  "term_id": "GO:0046471"
}